{
  "gene_name": "Ubiquitin-like protein ISG15",
  "gene_symbol": "ISG15",
  "term_id": "GO:0045087",
  "gene": "UniProtKB:P05161",
  "term_label": "innate immune response"
}